cholecystokinin receptor activity [GO:0004951] (molecular function) Definition: Combining with cholecystokinin and transmitting the signal across the membrane by activating an associated G-protein to initiate a change in cell activity. Cholecystokinin can act as a neuropeptide or as a gastrointestinal hormone. References: PMID:9835394 Sources: GOC:signaling Also known as: CCK receptor activity Relationships: is a type of G protein-coupled peptide receptor activity [GO:0008528]; BFO_0000050 cholecystokinin signaling pathway [GO:0038188]